{
  "term_label": "exocytosis",
  "gene_name": "Synaptosomal-associated protein 23",
  "gene_symbol": "SNAP23",
  "gene": "UniProtKB:O00161",
  "term_id": "GO:0006887"
}